voltage-gated monoatomic cation channel activity [GO:0022843] (molecular function) Subtypes: GO:0005245, voltage-gated potassium channel activity [GO:0005249], voltage-gated proton channel activity [GO:0030171] Relationships: is a type of voltage-gated monoatomic ion channel activity [GO:0005244]; is a type of monoatomic cation channel activity [GO:0005261] Sources: GOC:mtg_transport, ISBN:0815340729 Also known as: voltage-gated cation channel activity Definition: Enables the transmembrane transfer of a cation by a voltage-gated channel. A cation is a positively charged ion. A voltage-gated channel is a channel whose open state is dependent on the voltage across the membrane in which it is embedded.